{
  "term_label": "Unknown cellular component",
  "gene_name": "Hematopoietically-expressed homeobox protein HHEX",
  "gene_symbol": "HHEX",
  "gene": "UniProtKB:Q03014",
  "term_id": "UNKNOWN:0003"
}